glucose dehydrogenase (FAD, quinone) activity [GO:0140762] (molecular function) Definition: Catalysis of the reaction: a quinone + D-glucose = a quinol + D-glucono-1,5-lactone. Sources: RHEA:47372 Relationships: is a type of GO:0004344; is a type of GO:0016901